mRNA dihydrouridine synthase activity [GO:0106414] (molecular function) Relationships: is a type of RNA dihydrouridine synthase activity [GO:0106413] References: PMID:34798057 Definition: Catalysis of the reaction: mRNA-uracil + NAD(P)+ = mRNA-dihydrouridine + NAD(P)H+ + H+.